{
  "term_label": "Unknown cellular component",
  "gene_name": "3'-5' RNA helicase YTHDC2",
  "term_id": "UNKNOWN:0003",
  "gene": "UniProtKB:Q9H6S0",
  "gene_symbol": "YTHDC2"
}